geranylgeranyl diphosphate biosynthetic process [GO:0033386] (biological process) Also known as: geranylgeranyl diphosphate anabolism, geranylgeranyl diphosphate biosynthesis, geranylgeranyl diphosphate formation, geranylgeranyl diphosphate synthesis Sources: GOC:mah Definition: The chemical reactions and pathways resulting in the formation of geranylgeranyl diphosphate. Relationships: is a type of phospholipid biosynthetic process [GO:0008654]; is a type of terpenoid biosynthetic process [GO:0016114]; is a type of geranylgeranyl diphosphate metabolic process [GO:0033385]